{
  "term_id": "GO:0045165",
  "gene_name": "Transcription factor SOX-5",
  "term_label": "cell fate commitment",
  "gene": "UniProtKB:P35711",
  "gene_symbol": "SOX5"
}